{
  "gene_name": "Transmembrane protein 65",
  "gene": "UniProtKB:Q6PI78",
  "gene_symbol": "TMEM65",
  "term_label": "regulation of cardiac conduction",
  "term_id": "GO:1903779"
}